{
  "term_label": "central nervous system development",
  "gene_name": "Motor neuron and pancreas homeobox protein 1",
  "term_id": "GO:0007417",
  "gene_symbol": "MNX1",
  "gene": "UniProtKB:P50219"
}